nuclear steroid receptor activity [GO:0003707] (molecular function) Relationships: is a type of nuclear receptor activity [GO:0004879]; is part of nuclear receptor-mediated steroid hormone signaling pathway [GO:0030518] References: PMID:14708019 Sources: GOC:signaling Definition: A nuclear receptor activity regulated by steroid binding and modulating the transcription of specific gene sets transcribed by RNA polymerase II. Also known as: steroid hormone receptor activity Subtypes: nuclear glucocorticoid receptor activity [GO:0004883], nuclear estrogen receptor activity [GO:0030284]